{
  "gene": "UniProtKB:Q9NW61",
  "gene_name": "Pleckstrin homology domain-containing family J member 1",
  "term_label": "receptor recycling",
  "term_id": "GO:0001881",
  "gene_symbol": "PLEKHJ1"
}